{
  "gene_name": "Protein Wnt-8b",
  "gene": "UniProtKB:Q93098",
  "term_label": "extracellular space",
  "gene_symbol": "WNT8B",
  "term_id": "GO:0005615"
}